negative regulation of interleukin-18 production [GO:0032701] (biological process) References: PMID:23710316 Sources: GOC:mah Also known as: down regulation of interleukin-18 production, down-regulation of interleukin-18 production, downregulation of interleukin-18 production, negative regulation of IL-18 production, inhibition of interleukin-18 production, negative regulation of interleukin-18 biosynthetic process, negative regulation of interleukin-18 secretion Definition: Any process that stops, prevents, or reduces the frequency, rate, or extent of interleukin-18 production. Relationships: is a type of negative regulation of cytokine production [GO:0001818]; is_a regulation of interleukin-18 production [GO:0032661]; negatively regulates GO:0032621